{
  "gene": "UniProtKB:A0A0C5B5G6",
  "term_label": "DNA binding",
  "term_id": "GO:0003677",
  "gene_name": "Mitochondrial-derived peptide MOTS-c",
  "gene_symbol": "MT-RNR1"
}